protein O-linked glycosylation via galactose [GO:0180062] (biological process) Also known as: protein O-linked galactosylation Definition: A glycoprotein biosynthetic process starting with the covalent linkage of galactose via a beta-glycosidic bond to the oxygen atom of the hydroxyl group of a hydroxyproline, a hydroxylysine, a serine or a threonine in a protein, which can be further elongated with the sequential addition of sugar units resulting in the formation of a protein O-linked glycan. Hydroxylysine modification occurs in the endoplasmic reticulum and is predominantly found in collagen. Hydroxyproline modification occurs in the Golgi and is found only in plant proteins. Relationships: is a type of protein O-linked glycosylation [GO:0006493] References: PMID:17516569, PMID:30822656, PMID:33815452